{
  "gene": "UniProtKB:Q96A57",
  "gene_symbol": "TMEM230",
  "gene_name": "Transmembrane protein 230",
  "term_id": "GO:0012505",
  "term_label": "endomembrane system"
}